{
  "gene": "UniProtKB:P0DJG4",
  "term_label": "Unknown biological process",
  "gene_name": "Testicular haploid expressed gene protein-like",
  "gene_symbol": "THEGL",
  "term_id": "UNKNOWN:0002"
}